{
  "term_label": "regulation of signal transduction",
  "gene_symbol": "GRK5",
  "term_id": "GO:0009966",
  "gene_name": "G protein-coupled receptor kinase 5",
  "gene": "UniProtKB:P34947"
}